{
  "gene": "UniProtKB:O00159",
  "term_id": "GO:0015629",
  "gene_symbol": "MYO1C",
  "gene_name": "Unconventional myosin-Ic",
  "term_label": "actin cytoskeleton"
}